regulation of systemic arterial blood pressure involved in acute-phase response [GO:0002530] (biological process) Sources: GOC:jal, ISBN:081533642X Also known as: blood pressure regulation during acute phase response, regulation of systemic arterial blood pressure during acute phase response Definition: Any process that modulates the force with which blood travels through the circulatory system that contributes to the acute phase response. The acute phase response occurs during the early phases of an infection and is marked by changes in the production of plasma proteins such as C-reactive protein. Relationships: is a type of regulation of systemic arterial blood pressure [GO:0003073]; is part of acute-phase response [GO:0006953]